{
  "gene_name": "Aldo-keto reductase family 1 member C4",
  "gene": "UniProtKB:P17516",
  "gene_symbol": "AKR1C4",
  "term_id": "GO:0004032",
  "term_label": "aldose reductase (NADPH) activity"
}